{
  "gene_symbol": "ITGB5",
  "term_label": "stress fiber assembly",
  "gene": "UniProtKB:P18084",
  "gene_name": "Integrin beta-5",
  "term_id": "GO:0043149"
}